{
  "gene": "UniProtKB:Q63HQ0",
  "term_label": "AP-1 adaptor complex binding",
  "term_id": "GO:0035650",
  "gene_name": "AP-1 complex-associated regulatory protein",
  "gene_symbol": "AP1AR"
}